{
  "gene_symbol": "SEPTIN12",
  "gene_name": "Septin-12",
  "gene": "UniProtKB:Q8IYM1",
  "term_label": "septin complex",
  "term_id": "GO:0031105"
}